{
  "gene": "UniProtKB:Q53HL2",
  "term_label": "chromosome passenger complex",
  "term_id": "GO:0032133",
  "gene_symbol": "CDCA8",
  "gene_name": "Borealin"
}